7-epi-alpha-selinene synthase activity [GO:0102906] (molecular function) Relationships: is a type of carbon-oxygen lyase activity, acting on phosphates [GO:0016838] Definition: Catalysis of the reaction: 2-trans,6-trans-farnesyl diphosphate(3-) = (-)-7-epi-alpha-selinene + diphosphoric acid. Sources: EC:4.2.3.86, GOC:pz